protein N-acyltransferase activity [GO:0140186] (molecular function) Subtypes: protein N-acetyltransferase activity [GO:0034212] Relationships: is a type of N-acyltransferase activity [GO:0016410]; is a type of catalytic activity, acting on a protein [GO:0140096] Definition: Catalysis of the reaction: an acyl-CoA + L-lysyl-[protein] = N6-acyl-L-lysyl-[protein] + CoA + H+. Sources: RHEA:53916 Also known as: protein acyltransferase activity